{
  "gene_name": "Beta-synuclein",
  "term_id": "GO:0048488",
  "gene": "UniProtKB:Q16143",
  "term_label": "synaptic vesicle endocytosis",
  "gene_symbol": "SNCB"
}